{
  "gene": "UniProtKB:Q92633",
  "term_label": "neurogenesis",
  "gene_symbol": "LPAR1",
  "term_id": "GO:0022008",
  "gene_name": "Lysophosphatidic acid receptor 1"
}